{
  "gene_name": "Putative GTP-binding protein 6",
  "term_label": "ribosome binding",
  "gene_symbol": "GTPBP6",
  "gene": "UniProtKB:O43824",
  "term_id": "GO:0043022"
}